{
  "term_label": "ciliary basal body",
  "gene_symbol": "GAS8",
  "gene_name": "Dynein regulatory complex subunit 4",
  "gene": "UniProtKB:O95995",
  "term_id": "GO:0036064"
}